{
  "term_label": "positive regulation of sodium ion export across plasma membrane",
  "gene_symbol": "FXYD2",
  "gene": "UniProtKB:P54710",
  "term_id": "GO:1903278",
  "gene_name": "Sodium_potassium-transporting ATPase subunit gamma"
}